{
  "gene_symbol": "UBL4A",
  "term_label": "protein-folding chaperone binding",
  "term_id": "GO:0051087",
  "gene": "UniProtKB:P11441",
  "gene_name": "Ubiquitin-like protein 4A"
}